{
  "term_label": "proteasome-mediated ubiquitin-dependent protein catabolic process",
  "gene_symbol": "KLHL23",
  "gene_name": "Kelch-like protein 23",
  "term_id": "GO:0043161",
  "gene": "UniProtKB:Q8NBE8"
}